tRNA (L-threonylcarbamoyladenosine(37)-C2) methyltransferase activity [GO:0089715] (molecular function) Also known as: tRNA (L-threonylcarbamoyladenosine(37)-C(2)) methyltransferase activity, tRNA (L-threonylcarbamoyladenosine37-C2-) methyltransferase activity, tRNA m6t6A37 methyltransferase activity Definition: Catalysis of the reaction: S-adenosyl-L-methionine + tRNA containing N6-threonylcarbamoyladenosine at position 37 = S-adenosyl-L-homocysteine + tRNA containing N6-methylthreonylcarbamoyladenosine at position 37. Relationships: is a type of tRNA (adenine) methyltransferase activity [GO:0016426] Note: This activity is distinct from tRNA (adenine(37)-C2-)-methyltransferase activity (GO:0002935) in that it requires the presence of a threonylcarbamoyl modification. References: PMID:25063302 Sources: RHEA:70027